{
  "term_id": "UNKNOWN:0001",
  "gene_name": "T cell receptor alpha joining 44 (Fragment)",
  "gene": "UniProtKB:A0A075B6X8",
  "gene_symbol": "TRAJ44",
  "term_label": "Unknown molecular function"
}